histone H3S28 kinase activity [GO:0044022] (molecular function) Relationships: is a type of protein serine/threonine kinase activity [GO:0004674]; is a type of GO:0140996 Sources: GOC:jl Also known as: histone kinase activity (H3-S28 specific), histone serine kinase activity (H3-S28 specific), histone-serine kinase activity (H3-S28 specific) Definition: Catalysis of the reaction: histone H3-serine (position 28) + ATP = histone H3-phosphoserine (position 28) + ADP. This reaction is the addition of a phosphate group to the serine residue at position 28 of histone H3. Note: Comment: Note that the residue position corresponds to the canonical human H3 histone (UniProtKB:P84243); this residue is conserved across all eukaryotes, except for S. pombe. Residue 1 is the first residue following removal of the initiating Methionine (Met). Note that each histone is encoded by multiple genes, and sequences may vary across different genes within an organism.